activated SUMO-E1 ligase complex [GO:1990354] (cellular component) Relationships: is a type of SUMO ligase complex [GO:0106068]; is a type of nuclear protein-containing complex [GO:0140513]; has part GO:0031510 Also known as: SUMO-SAE1/2 complex Note: An example of this is SAE1 in human (UniProt symbol Q9UBE0) in PMID:15660128 (inferred from direct assay). Definition: A protein complex consisting of a SUMO protein bound to a SUMO activating enzyme complex. Activation by the E1 complex and linkage to the E2 enzyme UBE2I is required for the formation of covalent bonds between SUMO and its ultimate target proteins. References: PMID:15660128 Sources: GOC:bhm